{
  "gene_name": "GTPase IMAP family member 8",
  "term_label": "Unknown biological process",
  "gene": "UniProtKB:Q8ND71",
  "term_id": "UNKNOWN:0002",
  "gene_symbol": "GIMAP8"
}